{
  "term_id": "GO:0006954",
  "gene": "UniProtKB:Q99616",
  "gene_name": "C-C motif chemokine 13",
  "gene_symbol": "CCL13",
  "term_label": "inflammatory response"
}